{
  "term_id": "GO:0007186",
  "gene_symbol": "DEPTOR",
  "term_label": "G protein-coupled receptor signaling pathway",
  "gene_name": "DEP domain-containing mTOR-interacting protein",
  "gene": "UniProtKB:Q8TB45"
}